endosome to melanosome transport [GO:0035646] (biological process) Definition: The directed movement of substances from endosomes to the melanosome, a specialised lysosome-related organelle. Relationships: is a type of GO:0043485 References: PMID:16162817